cord factor receptor activity [GO:1990725] (molecular function) Also known as: TMD receptor activity, trehalose 6,6'-dimycolate receptor activity References: PMID:23602766 Sources: GOC:hjd Relationships: is a type of signaling receptor activity [GO:0038023] Definition: Combining with a cord factor, an M. tuberculosis cell wall glycolipid, and transmitting a signal from one side of the membrane to the other to initiate a change in cell activity.